{
  "term_id": "GO:0005634",
  "gene": "UniProtKB:Q9BXW9",
  "term_label": "nucleus",
  "gene_symbol": "FANCD2",
  "gene_name": "Fanconi anemia group D2 protein"
}